{
  "term_id": "GO:0003400",
  "gene": "UniProtKB:Q9HCU5",
  "gene_symbol": "PREB",
  "gene_name": "Prolactin regulatory element-binding protein",
  "term_label": "regulation of COPII vesicle coating"
}